neuromast primordium migration [GO:0048883] (biological process) References: PMID:15018940, PMID:15832385 Also known as: lateral line primordium migration Subtypes: GO:0048900, posterior lateral line neuromast primordium migration [GO:0048920] Definition: The migration of a cluster of a relatively undifferentiated cell originating at specific cephalic placodes and depositing proneuromasts along a developing lateral line, from which the neuromasts will develop. Relationships: is a type of cell migration [GO:0016477]; is part of lateral line development [GO:0048882]